{
  "term_id": "GO:0007409",
  "term_label": "axonogenesis",
  "gene_name": "Amyloid beta precursor like protein 1",
  "gene_symbol": "APLP1",
  "gene": "UniProtKB:P51693"
}